{
  "term_label": "Unknown molecular function",
  "gene_name": "RNA-binding protein PNO1",
  "term_id": "UNKNOWN:0001",
  "gene_symbol": "PNO1",
  "gene": "UniProtKB:Q9NRX1"
}